DNA-1,N6-ethenoadenine N-glycosylase activity [GO:0052820] (molecular function) Relationships: is a type of alkylbase DNA N-glycosylase activity [GO:0003905] References: PMID:21960007 Also known as: 1,N(6)-ethenoadenine N-glycosylase activity, 1,N6-ethenoadenine glycosylase activity Definition: Catalysis of the reaction: DNA with 1-N6-ethenoadenine + H2O = DNA with abasic site + 1-N6-ethenoadenine. This reaction is the removal of 1,N6-ethenoadenine by cleaving the N-C1' glycosidic bond between the target damaged DNA base and the deoxyribose sugar.